hydroxycinnamate 4-beta-glucosyltransferase activity [GO:0047218] (molecular function) Sources: EC:2.4.1.126 Relationships: is a type of GO:0035251 Definition: Catalysis of the reaction: 4-coumarate + UDP-D-glucose = 4-O-beta-D-glucosyl-4-hydroxycinnamate + UDP. Also acts on ferulate, caffeate and sinapate, forming a mixture of 4-glucosides and glucose esters. Also known as: UDP-glucose-hydroxycinnamate glucosyltransferase activity, UDP-glucose:trans-4-hydroxycinnamate 4-O-beta-D-glucosyltransferase activity, UDPglucose:trans-4-hydroxycinnamate 4-O-beta-D-glucosyltransferase activity, hydroxycinnamoyl glucosyltransferase activity, uridine diphosphoglucose-hydroxycinnamate glucosyltransferase activity